{
  "gene": "UniProtKB:Q93045",
  "term_id": "GO:0015631",
  "gene_name": "Stathmin-2",
  "gene_symbol": "STMN2",
  "term_label": "tubulin binding"
}